{
  "term_label": "late endosome to vacuole transport",
  "gene_name": "Charged multivesicular body protein 1b",
  "gene": "UniProtKB:Q7LBR1",
  "term_id": "GO:0045324",
  "gene_symbol": "CHMP1B"
}